{
  "gene_name": "Ubiquitin carboxyl-terminal hydrolase 17-like protein 13",
  "gene": "UniProtKB:C9JLJ4",
  "gene_symbol": "USP17L13",
  "term_id": "GO:0042981",
  "term_label": "regulation of apoptotic process"
}